{
  "term_id": "GO:0030688",
  "gene_name": "RNA-binding protein NOB1",
  "term_label": "preribosome, small subunit precursor",
  "gene": "UniProtKB:Q9ULX3",
  "gene_symbol": "NOB1"
}